cannabinoid signaling pathway [GO:0038171] (biological process) Subtypes: endocannabinoid signaling pathway [GO:0071926] Relationships: is a type of GO:0007186; BFO_0000051 GO:0004949 Sources: GOC:bf, GOC:jc, GOC:signaling, Wikipedia:Cannabinoid Definition: A G protein-coupled receptor signaling pathway initiated by a cannabinoid binding to its receptor on the cell surface, and ending with the regulation of a downstream cellular process, e.g. transcription. Cannabinoids are a class of diverse chemical compounds that include the endocannabinoids and the phytocannabinoids. Also known as: cannabinoid receptor signaling pathway, cannabinoid-activated signaling pathway, cannabinoid-mediated signaling pathway